negative regulation of secondary cell septum biogenesis [GO:1903396] (biological process) Definition: Any process that stops, prevents or reduces the frequency, rate or extent of secondary cell septum biogenesis. Relationships: is a type of negative regulation of mitotic division septum assembly [GO:0140280]; is a type of regulation of secondary cell septum biogenesis [GO:1903395]; negatively regulates secondary cell septum biogenesis [GO:1990344] References: PMID:23878277 Sources: GOC:TermGenie, GOC:di, GO_REF:0000058 Also known as: down regulation of secondary cell septum biogenesis, down-regulation of secondary cell septum biogenesis, downregulation of secondary cell septum biogenesis, inhibition of secondary cell septum biogenesis